{
  "gene": "UniProtKB:Q6NZI2",
  "term_id": "GO:0006361",
  "gene_name": "Caveolae-associated protein 1",
  "gene_symbol": "CAVIN1",
  "term_label": "transcription initiation at RNA polymerase I promoter"
}